positive regulation of formation of translation initiation ternary complex [GO:1901192] (biological process) Sources: GOC:TermGenie Relationships: is a type of positive regulation of protein-containing complex assembly [GO:0031334]; is a type of regulation of formation of translation initiation ternary complex [GO:1901190]; positively regulates GO:0001677 Also known as: activation of translation initiation ternary complex assembly, positive regulation of translation initiation ternary complex assembly, up regulation of formation of translation initiation ternary complex, up regulation of translation initiation ternary complex assembly, up-regulation of formation of translation initiation ternary complex, up-regulation of translation initiation ternary complex assembly, upregulation of formation of translation initiation ternary complex, upregulation of translation initiation ternary complex assembly, activation of formation of translation initiation ternary complex Definition: Any process that activates or increases the frequency, rate or extent of formation of translation initiation ternary complex.